{
  "gene_symbol": "TMCO3",
  "term_label": "Unknown biological process",
  "gene": "UniProtKB:Q6UWJ1",
  "gene_name": "Transmembrane and coiled-coil domain-containing protein 3",
  "term_id": "UNKNOWN:0002"
}